positive regulation of cellular response to phosphate starvation [GO:0080040] (biological process) Definition: Any process that activates or increases the frequency, rate or extent of cellular response to phosphate starvation. Relationships: is a type of positive regulation of response to nutrient levels [GO:0032109]; is_a positive regulation of cellular process [GO:0048522]; is a type of regulation of cellular response to phosphate starvation [GO:0140255]; positively regulates GO:0016036 References: PMID:18315545